negative regulation of protein depolymerization [GO:1901880] (biological process) Definition: Any process that stops, prevents or reduces the frequency, rate or extent of protein depolymerization. References: PMID:12032137 Sources: GOC:BHF, GOC:TermGenie, GOC:rl Subtypes: negative regulation of microtubule depolymerization [GO:0007026], negative regulation of actin filament depolymerization [GO:0030835], negative regulation of intermediate filament depolymerization [GO:0030843], GO:1903389 Relationships: is a type of negative regulation of protein-containing complex disassembly [GO:0043242]; is a type of regulation of protein depolymerization [GO:1901879]; negatively regulates GO:0051261 Also known as: down regulation of protein depolymerization, down regulation of protein polymer breakdown, down regulation of protein polymer catabolic process, down regulation of protein polymer catabolism, down regulation of protein polymer degradation, down-regulation of protein depolymerization, down-regulation of protein polymer breakdown, down-regulation of protein polymer catabolic process, down-regulation of protein polymer catabolism, down-regulation of protein polymer degradation, downregulation of protein depolymerization, downregulation of protein polymer breakdown, downregulation of protein polymer catabolic process, downregulation of protein polymer catabolism, downregulation of protein polymer degradation, inhibition of protein polymer breakdown, inhibition of protein polymer catabolic process, inhibition of protein polymer catabolism, inhibition of protein polymer degradation, negative regulation of protein polymer breakdown, negative regulation of protein polymer catabolic process, negative regulation of protein polymer catabolism, negative regulation of protein polymer degradation, inhibition of protein depolymerization